{
  "term_label": "P-type calcium transporter activity",
  "gene_symbol": "ATP2B1",
  "gene": "UniProtKB:P20020",
  "term_id": "GO:0005388",
  "gene_name": "Plasma membrane calcium-transporting ATPase 1"
}